{
  "gene_name": "Chymotrypsin-like elastase family member 1",
  "gene_symbol": "CELA1",
  "gene": "UniProtKB:Q9UNI1",
  "term_id": "GO:0004252",
  "term_label": "serine-type endopeptidase activity"
}